{
  "gene_symbol": "LAT",
  "gene_name": "Linker for activation of T-cells family member 1",
  "gene": "UniProtKB:O43561",
  "term_label": "regulation of T cell activation",
  "term_id": "GO:0050863"
}